{
  "gene": "UniProtKB:Q15078",
  "term_id": "GO:0007420",
  "term_label": "brain development",
  "gene_symbol": "CDK5R1",
  "gene_name": "Cyclin-dependent kinase 5 activator 1"
}